{
  "term_label": "Unknown cellular component",
  "gene_symbol": "RPIA",
  "gene_name": "Ribose-5-phosphate isomerase",
  "gene": "UniProtKB:P49247",
  "term_id": "UNKNOWN:0003"
}